{
  "term_label": "nucleus",
  "gene": "UniProtKB:Q96PZ2",
  "term_id": "GO:0005634",
  "gene_name": "Serine protease FAM111A",
  "gene_symbol": "FAM111A"
}